{
  "gene": "UniProtKB:P16435",
  "term_label": "response to hormone",
  "gene_symbol": "POR",
  "term_id": "GO:0009725",
  "gene_name": "NADPH--cytochrome P450 reductase"
}